peptidyl-selenocysteine modification [GO:0050844] (biological process) Definition: The modification of peptidyl-selenocysteine. Relationships: is a type of peptidyl-amino acid modification [GO:0018193] Sources: GOC:ai